{
  "term_id": "GO:0000381",
  "gene_name": "RNA binding protein fox-1 homolog 3",
  "term_label": "regulation of alternative mRNA splicing, via spliceosome",
  "gene": "UniProtKB:A6NFN3",
  "gene_symbol": "RBFOX3"
}